{
  "gene_name": "GDP-D-glucose phosphorylase 1",
  "term_label": "glucose metabolic process",
  "gene_symbol": "GDPGP1",
  "gene": "UniProtKB:Q6ZNW5",
  "term_id": "GO:0006006"
}